negative regulation of G protein-coupled receptor signaling pathway [GO:0045744] (BP) Definition: Any process that stops, prevents, or reduces the frequency, rate or extent of G protein-coupled receptor signaling pathway. Sources: GOC:go_curators Also known as: down regulation of G-protein coupled receptor protein signaling pathway, down-regulation of G-protein coupled receptor protein signaling pathway, downregulation of G-protein coupled receptor protein signaling pathway, negative regulation of G protein coupled receptor protein signaling pathway, negative regulation of G protein coupled receptor protein signalling pathway, negative regulation of G-protein coupled receptor protein signaling pathway, negative regulation of G-protein coupled receptor protein signalling pathway, negative regulation of G-protein-coupled receptor protein signalling pathway, negative regulation of GPCR protein signaling pathway, negative regulation of GPCR protein signalling pathway, inhibition of G-protein coupled receptor protein signaling pathway Relationships: is a type of regulation of G protein-coupled receptor signaling pathway [GO:0008277]; is_a negative regulation of signal transduction [GO:0009968]; RO_0002212 G protein-coupled receptor signaling pathway [GO:0007186] Subtypes: GO:0002029, negative regulation of opsin-mediated signaling pathway [GO:0016059], termination of G protein-coupled receptor signaling pathway [GO:0038032], GO:0060160, negative regulation of adenosine receptor signaling pathway [GO:0060169], negative regulation of chemokine-mediated signaling pathway [GO:0070100], negative regulation of thrombin-activated receptor signaling pathway [GO:0070495], GO:0106072, negative regulation of angiotensin-activated signaling pathway [GO:0110062], negative regulation of phospholipase C-activating G protein-coupled receptor signaling pathway [GO:1900737], G protein-coupled receptor catabolic process [GO:1990172], negative regulation of octopamine or tyramine signaling pathway [GO:2000126], negative regulation of opioid receptor signaling pathway [GO:2000475]